negative regulation of conidium formation [GO:0075308] (biological process) Relationships: is a type of negative regulation of cell development [GO:0010721]; is a type of negative regulation of sporulation [GO:0043939]; is a type of regulation of conidium formation [GO:0075306]; is a type of negative regulation of asexual reproduction [GO:1903665]; negatively regulates conidium formation [GO:0048315] Definition: Any process that stops, prevents, or reduces the frequency, rate or extent of conidium formation, a process of producing non-motile spores, called conidia, via mitotic asexual reproduction in higher fungi. Conidia are haploid cells genetically identical to their haploid parent. They are produced by conversion of hyphal elements, or are borne on sporogenous cells on or within specialized structures termed conidiophores, and participate in dispersal of the fungus. Sources: GOC:di, GOC:pamgo_curators